ligand-gated calcium channel activity [GO:0099604] (molecular function) Definition: Enables the transmembrane transfer of a calcium ions by a channel that opens when a specific ligand has been bound by the channel complex or one of its constituent parts. Sources: GOC:dos Relationships: is_a calcium channel activity [GO:0005262]; is a type of GO:0099094; is part of GO:0019722 Subtypes: intracellularly gated calcium channel activity [GO:0015278], glutamate-gated calcium ion channel activity [GO:0022849], pH-gated calcium channel activity [GO:0160126]